{
  "term_id": "GO:0007052",
  "term_label": "mitotic spindle organization",
  "gene_name": "Dynactin subunit 6",
  "gene": "UniProtKB:O00399",
  "gene_symbol": "DCTN6"
}